{
  "gene_name": "Cyclin-T1",
  "gene_symbol": "CCNT1",
  "gene": "UniProtKB:O60563",
  "term_label": "nucleus",
  "term_id": "GO:0005634"
}